stem cell factor receptor activity [GO:0005020] (molecular function) Definition: Combining with stem cell factor (SCF) receptor ligand and transmitting the signal from one side of the membrane to the other to initiate a change in cell activity by catalysis of the reaction: ATP + a protein-L-tyrosine = ADP + a protein-L-tyrosine phosphate. Stem cell factor is a cytokine that stimulates mast cell growth and differentiation. References: PMID:10698217 Sources: GOC:jl, GOC:signaling Relationships: is a type of transmembrane receptor protein tyrosine kinase activity [GO:0004714]; is part of Kit signaling pathway [GO:0038109] Also known as: KIT ligand receptor activity, KL receptor activity, SCF receptor activity, KIT